organic phosphonate transport [GO:0015716] (biological process) Definition: The directed movement of phosphonates into, out of or within a cell, or between cells, by means of some agent such as a transporter or pore. A phosphonate is any salt, anion, or ester of phosphonic acid (HPO(OH)2). Sources: GOC:krc Relationships: is a type of inorganic anion transport [GO:0015698] Also known as: alkylphosphonate transport